{
  "term_label": "catalytic step 2 spliceosome",
  "term_id": "GO:0071013",
  "gene": "UniProtKB:O60508",
  "gene_name": "Pre-mRNA-processing factor 17",
  "gene_symbol": "CDC40"
}